{
  "gene_name": "WAP four-disulfide core domain protein 12",
  "gene_symbol": "WFDC12",
  "term_label": "antibacterial humoral response",
  "gene": "UniProtKB:Q8WWY7",
  "term_id": "GO:0019731"
}